{
  "gene_name": "Cathepsin B",
  "term_label": "cysteine-type endopeptidase activity",
  "gene": "UniProtKB:P07858",
  "term_id": "GO:0004197",
  "gene_symbol": "CTSB"
}